T=28 icosahedral capsid [GO:0160171] (cellular component) Definition: The protein coat that surrounds the infective nucleic acid in some virus particles where the subunits (capsomeres) are arranged to form an icosahedron with T=28 symmetry. Sources: VZ:6057 Relationships: is a type of icosahedral viral capsid [GO:0019030]